{
  "gene": "UniProtKB:Q9Y5F1",
  "term_id": "GO:0005886",
  "gene_symbol": "PCDHB12",
  "gene_name": "Protocadherin beta-12",
  "term_label": "plasma membrane"
}